interleukin-8-mediated signaling pathway [GO:0038112] (biological process) Relationships: is a type of GO:0019221; is part of cellular response to interleukin-8 [GO:0098759] Also known as: IL-8-mediated signaling pathway, interleukin-8-mediated signalling pathway Definition: The series of molecular signals initiated by interleukin-8 binding to its receptor on the surface of a cell, and ending with the regulation of a downstream cellular process, e.g. transcription. Sources: GOC:nhn, GOC:signaling